water-soluble vitamin biosynthetic process [GO:0042364] (biological process) Subtypes: biotin biosynthetic process [GO:0009102], GO:0009231, GO:0009236, pantothenate biosynthetic process [GO:0015940], GO:0019853, thiamine-containing compound biosynthetic process [GO:0042724], vitamin B6 biosynthetic process [GO:0042819], folic acid biosynthetic process [GO:0046656] Also known as: water-soluble vitamin anabolism, water-soluble vitamin biosynthesis, water-soluble vitamin formation, water-soluble vitamin synthesis Sources: GOC:jl Relationships: is a type of GO:0009110 Definition: The chemical reactions and pathways resulting in the formation of any of a diverse group of vitamins that are soluble in water.